{
  "gene_name": "Cytochrome P450 4F11",
  "term_label": "menaquinone catabolic process",
  "term_id": "GO:0042361",
  "gene": "UniProtKB:Q9HBI6",
  "gene_symbol": "CYP4F11"
}